{
  "gene_name": "Melanophilin",
  "gene": "UniProtKB:Q9BV36",
  "gene_symbol": "MLPH",
  "term_label": "myosin binding",
  "term_id": "GO:0017022"
}